{
  "gene_symbol": "SEPTIN3",
  "term_id": "GO:0060090",
  "term_label": "molecular adaptor activity",
  "gene": "UniProtKB:Q9UH03",
  "gene_name": "Neuronal-specific septin-3"
}